{
  "gene": "UniProtKB:Q8NFY4",
  "term_id": "GO:0030335",
  "term_label": "positive regulation of cell migration",
  "gene_name": "Semaphorin-6D",
  "gene_symbol": "SEMA6D"
}